{
  "gene_symbol": "SNTG1",
  "gene_name": "Gamma-1-syntrophin",
  "term_label": "dystrophin-associated glycoprotein complex",
  "gene": "UniProtKB:Q9NSN8",
  "term_id": "GO:0016010"
}